{
  "gene": "UniProtKB:Q9Y232",
  "term_id": "GO:0061628",
  "gene_symbol": "CDYL",
  "term_label": "histone H3K27me3 reader activity",
  "gene_name": "Chromodomain Y-like protein"
}